{
  "gene_name": "F-box_WD repeat-containing protein 11",
  "term_label": "vesicle transport along microtubule",
  "gene_symbol": "FBXW11",
  "term_id": "GO:0047496",
  "gene": "UniProtKB:Q9UKB1"
}